{
  "term_label": "plasma membrane",
  "gene_name": "Oxysterol-binding protein-related protein 2",
  "term_id": "GO:0005886",
  "gene": "UniProtKB:Q9H1P3",
  "gene_symbol": "OSBPL2"
}